{
  "term_id": "GO:0045109",
  "gene": "UniProtKB:Q7Z3Y8",
  "term_label": "intermediate filament organization",
  "gene_symbol": "KRT27",
  "gene_name": "Keratin, type I cytoskeletal 27"
}